{
  "gene": "UniProtKB:Q8N660",
  "term_label": "Unknown cellular component",
  "term_id": "UNKNOWN:0003",
  "gene_symbol": "NBPF15",
  "gene_name": "Neuroblastoma breakpoint family member 15"
}